GU repeat RNA binding [GO:1990605] (molecular function) References: PMID:20081200 Definition: Binding to an RNA molecule containing GU repeats. Relationships: is a type of RNA binding [GO:0003723]